{
  "term_label": "Unknown molecular function",
  "gene_name": "Tetratricopeptide repeat protein 39C",
  "term_id": "UNKNOWN:0001",
  "gene": "UniProtKB:Q8N584",
  "gene_symbol": "TTC39C"
}